methanogenesis, from methanol [GO:0019387] (biological process) Subtypes: methane biosynthetic process from methanol and hydrogen [GO:1990491] Sources: GOC:ai Relationships: is a type of methanol metabolic process [GO:0015945]; is_a methanogenesis [GO:0015948] Also known as: methane biosynthesis from methanol, methane biosynthetic process from methanol Definition: The formation of methane, a colorless, odorless, flammable gas with the formula CH4, from other components, including methanol.